{
  "gene_symbol": "TREX1",
  "gene_name": "Three-prime repair exonuclease 1",
  "gene": "UniProtKB:Q9NSU2",
  "term_id": "GO:0005737",
  "term_label": "cytoplasm"
}